{
  "term_label": "response to exogenous dsRNA",
  "term_id": "GO:0043330",
  "gene_name": "Interferon alpha-6",
  "gene": "UniProtKB:P05013",
  "gene_symbol": "IFNA6"
}